symbiont entry into host cell via disruption of host cell envelope [GO:0098994] (biological process) Sources: GOC:dos Definition: The disruption by a symbiont of host cell envelope components to allow entry into the host cell. Also known as: disruption of host cell envelope during viral entry Relationships: is a type of symbiont-mediated disruption of host cell envelope [GO:0098933]; is part of symbiont entry into host cell [GO:0046718]